fumagillin biosynthetic process [GO:1902086] (biological process) Definition: The chemical reactions and pathways resulting in the formation of fumagillin. References: PMID:23488861 Sources: GOC:TermGenie, GOC:di Also known as: fumagillin anabolism, fumagillin biosynthesis, fumagillin formation, fumagillin synthesis Relationships: is a type of secondary metabolic process [GO:0019748]; is a type of monocarboxylic acid biosynthetic process [GO:0072330]; is a type of epoxide metabolic process [GO:0097176]; is a type of ether biosynthetic process [GO:1901503] Regulation: regulated by regulation of fumagillin biosynthetic process [GO:1902090]; negatively regulated by GO:1902091; positively regulated by positive regulation of fumagillin biosynthetic process [GO:1902092]